negative regulation of B-1 B cell differentiation [GO:0001925] (biological process) Sources: GOC:add, ISBN:0781735149 Also known as: down regulation of B-1 B cell differentiation, down-regulation of B-1 B cell differentiation, downregulation of B-1 B cell differentiation, negative regulation of B-1 B lymphocyte differentiation, negative regulation of B-1 B-cell differentiation, negative regulation of B-1 B-lymphocyte differentiation, inhibition of B-1 B cell differentiation, negative regulation of B-1 B cell development Relationships: is a type of GO:0001924; is_a negative regulation of B cell differentiation [GO:0045578]; negatively regulates B-1 B cell differentiation [GO:0001923] Note: Note that immunologists typically use the word 'development' to refer to cells of B or T cell lineages undergoing the process that GO describes as 'cell differentiation'. Definition: Any process that stops, prevents, or reduces the rate of B-1 B cell differentiation.